{
  "gene_name": "CUB domain-containing protein 1",
  "gene_symbol": "CDCP1",
  "gene": "UniProtKB:Q9H5V8",
  "term_id": "UNKNOWN:0002",
  "term_label": "Unknown biological process"
}